{
  "gene_name": "HLA class II histocompatibility antigen, DQ beta 1 chain",
  "term_id": "GO:0005765",
  "gene_symbol": "HLA-DQB1",
  "gene": "UniProtKB:P01920",
  "term_label": "lysosomal membrane"
}